{
  "gene": "UniProtKB:A1A5D9",
  "term_label": "Unknown molecular function",
  "gene_symbol": "BICDL2",
  "gene_name": "BICD family-like cargo adapter 2",
  "term_id": "UNKNOWN:0001"
}